{
  "gene_symbol": "CGAS",
  "term_label": "double-stranded DNA binding",
  "term_id": "GO:0003690",
  "gene_name": "Cyclic GMP-AMP synthase",
  "gene": "UniProtKB:Q8N884"
}